{
  "term_label": "Unknown cellular component",
  "gene_symbol": "SCYGR6",
  "gene_name": "Small cysteine and glycine repeat-containing protein 6",
  "term_id": "UNKNOWN:0003",
  "gene": "UniProtKB:A0A286YF77"
}